{
  "gene_name": "Zinc finger protein 860",
  "gene_symbol": "ZNF860",
  "term_label": "nucleus",
  "term_id": "GO:0005634",
  "gene": "UniProtKB:A6NHJ4"
}